negative regulation of cellular response to insulin stimulus [GO:1900077] (biological process) Also known as: down regulation of cellular response to insulin stimulus, down-regulation of cellular response to insulin stimulus, downregulation of cellular response to insulin stimulus, inhibition of cellular response to insulin stimulus Definition: Any process that stops, prevents or reduces the frequency, rate or extent of cellular response to insulin stimulus. Relationships: is a type of negative regulation of cellular process [GO:0048523]; is a type of negative regulation of response to stimulus [GO:0048585]; is a type of regulation of cellular response to insulin stimulus [GO:1900076]; negatively regulates GO:0032869 Subtypes: GO:0046627 Sources: GOC:TermGenie, GOC:yaf